{
  "gene_name": "High affinity nerve growth factor receptor",
  "gene": "UniProtKB:P04629",
  "term_id": "GO:0007169",
  "term_label": "cell surface receptor protein tyrosine kinase signaling pathway",
  "gene_symbol": "NTRK1"
}